{
  "term_label": "sodium:iodide symporter activity",
  "gene_symbol": "SLC5A5",
  "term_id": "GO:0008507",
  "gene_name": "Sodium_iodide cotransporter",
  "gene": "UniProtKB:Q92911"
}